{
  "gene": "UniProtKB:Q13099",
  "gene_name": "Intraflagellar transport protein 88 homolog",
  "gene_symbol": "IFT88",
  "term_id": "GO:0005814",
  "term_label": "centriole"
}